{
  "gene_symbol": "LIG1",
  "term_label": "Okazaki fragment processing involved in mitotic DNA replication",
  "gene": "UniProtKB:P18858",
  "gene_name": "DNA ligase 1",
  "term_id": "GO:1903461"
}